response to norepinephrine [GO:0071873] (biological process) Note: Note that epinephrine and norepinephrine are ligands for the same receptors, and there are multiple adrenergic receptors. Relationships: is a type of response to catecholamine [GO:0071869] Also known as: response to noradrenaline stimulus, response to norepinephrine stimulus Definition: Any process that results in a change in state or activity of a cell or an organism (in terms of movement, secretion, enzyme production, gene expression, etc.) as a result of a norepinephrine stimulus. Norepinephrine is a catecholamine that has the formula C8H11NO3; it acts as a hormone, and as a neurotransmitter in most of the sympathetic nervous system. Sources: GOC:BHF, GOC:mah Subtypes: GO:0071874